{
  "term_label": "Unknown molecular function",
  "gene": "UniProtKB:Q5H9L2",
  "gene_name": "Transcription elongation factor A protein-like 5",
  "term_id": "UNKNOWN:0001",
  "gene_symbol": "TCEAL5"
}